{
  "term_id": "GO:0072544",
  "term_label": "L-DOPA binding",
  "gene": "UniProtKB:P51810",
  "gene_symbol": "GPR143",
  "gene_name": "G-protein coupled receptor 143"
}